{
  "gene": "UniProtKB:Q8NBQ5",
  "term_label": "oxidoreductase activity, acting on the CH-OH group of donors, NAD or NADP as acceptor",
  "gene_name": "Estradiol 17-beta-dehydrogenase 11",
  "term_id": "GO:0016616",
  "gene_symbol": "HSD17B11"
}